{
  "gene_name": "Centromere protein I",
  "term_id": "UNKNOWN:0001",
  "gene_symbol": "CENPI",
  "gene": "UniProtKB:Q92674",
  "term_label": "Unknown molecular function"
}